{
  "term_id": "GO:0022008",
  "term_label": "neurogenesis",
  "gene_symbol": "FGF7",
  "gene": "UniProtKB:P21781",
  "gene_name": "Fibroblast growth factor 7"
}